{
  "term_id": "UNKNOWN:0001",
  "gene": "UniProtKB:Q8TEF2",
  "gene_symbol": "C10orf105",
  "term_label": "Unknown molecular function",
  "gene_name": "Uncharacterized protein C10orf105"
}